{
  "term_label": "late endosome",
  "gene_name": "Ankyrin repeat domain-containing protein 13D",
  "gene": "UniProtKB:Q6ZTN6",
  "term_id": "GO:0005770",
  "gene_symbol": "ANKRD13D"
}